{
  "gene_symbol": "RSPH1",
  "term_label": "sperm flagellum",
  "term_id": "GO:0036126",
  "gene_name": "Radial spoke head 1 homolog",
  "gene": "UniProtKB:Q8WYR4"
}